complement component iC3b receptor activity [GO:0001858] (molecular function) Definition: Combining with the iC3b product of the complement cascade and transmitting the signal from one side of the membrane to the other to initiate a change in cell activity. Sources: GOC:add, GOC:signaling, ISBN:0781735149 Relationships: is a type of GO:0001847; is_a complement receptor activity [GO:0004875]; has part complement component iC3b binding [GO:0001852]